{
  "gene_symbol": "SEMA3C",
  "gene_name": "Semaphorin-3C",
  "gene": "UniProtKB:Q99985",
  "term_id": "GO:0005886",
  "term_label": "plasma membrane"
}